negative regulation of adenylate cyclase-activating adrenergic receptor signaling pathway [GO:0071878] (biological process) Definition: Any process that stops, prevents, or reduces the frequency, rate or extent of an adenylate cyclase-activating adrenergic receptor protein signaling pathway activity. An adrenergic receptor signaling pathway is the series of molecular signals generated as a consequence of an adrenergic receptor binding to one of its physiological ligands. Sources: GOC:BHF, GOC:mah Relationships: is a type of negative regulation of adenylate cyclase-activating G protein-coupled receptor signaling pathway [GO:0106072]; negatively regulates GO:0071880 Also known as: negative regulation of adrenergic receptor signaling pathway, negative regulation of adrenergic receptor signalling pathway Subtypes: GO:0140199